{
  "term_id": "GO:0007020",
  "gene_symbol": "NDE1",
  "gene_name": "Nuclear distribution protein nudE homolog 1",
  "term_label": "microtubule nucleation",
  "gene": "UniProtKB:Q9NXR1"
}